nicotinate nucleotide salvage [GO:0019358] (biological process) Definition: The generation of nicotinate nucleotide without de novo synthesis. Also known as: nicotinate nucleotide biosynthesis, salvage pathway, nicotinate nucleotide biosynthetic process, salvage pathway Relationships: is a type of nicotinate nucleotide biosynthetic process [GO:0019357]; is_a pyridine nucleotide salvage [GO:0019365] Sources: GOC:go_curators